{
  "gene": "UniProtKB:P50552",
  "gene_symbol": "VASP",
  "gene_name": "Vasodilator-stimulated phosphoprotein",
  "term_label": "plasma membrane",
  "term_id": "GO:0005886"
}